{
  "gene_name": "Acyl-coenzyme A thioesterase 1",
  "gene_symbol": "ACOT1",
  "term_label": "acyl-CoA metabolic process",
  "gene": "UniProtKB:Q86TX2",
  "term_id": "GO:0006637"
}